{
  "gene": "UniProtKB:Q7RTM1",
  "term_id": "GO:0045299",
  "gene_symbol": "OTOP1",
  "term_label": "otolith mineralization",
  "gene_name": "Proton channel OTOP1"
}